{
  "term_id": "GO:0030865",
  "gene": "UniProtKB:O94844",
  "gene_symbol": "RHOBTB1",
  "gene_name": "Rho-related BTB domain-containing protein 1",
  "term_label": "cortical cytoskeleton organization"
}